epithelial cilium movement involved in determination of left/right asymmetry [GO:0060287] (biological process) Definition: The movement of cilia of epithelial cells of the Left Right Organizer (LRO), also referred to as the node in mouse or the Kupffer's vesicle in zebrafish, resulting in the leftward fluid flow across the LRO and generation or transport of a signal which determines asymmetry in an organism's body plan with respect to the left and right halves. Relationships: is a type of epithelial cilium movement involved in extracellular fluid movement [GO:0003351]; is part of determination of left/right symmetry [GO:0007368] Also known as: cilium movement involved in determinationof L/R asymmetry, Kuppfer's vesicle cilium movement involved in determination of left/right asymmetry, nodal cilium movement involved in determination of left/right asymmetry References: PMID:28559696, PMID:29367579 Sources: GOC:dgh, GOC:dph, GOC:krc, GOC:mlg